{
  "gene": "UniProtKB:Q13823",
  "term_label": "nucleolus",
  "term_id": "GO:0005730",
  "gene_name": "Nucleolar GTP-binding protein 2",
  "gene_symbol": "GNL2"
}